ubiquitin-dependent protein catabolic process via the N-end rule pathway [GO:0071596] (biological process) Also known as: ubiquitin-dependent protein breakdown via the N-end rule pathway, ubiquitin-dependent protein catabolism via the N-end rule pathway, ubiquitin-dependent protein degradation via the N-end rule pathway Definition: The chemical reactions and pathways resulting in the breakdown of a protein or peptide covalently tagged with ubiquitin, via the N-end rule pathway. In the N-end rule pathway, destabilizing N-terminal residues (N-degrons) in substrates are recognized by E3 ligases (N-recognins), whereupon the substrates are linked to ubiquitin and then delivered to the proteasome for degradation. References: PMID:19246002, PMID:9112437 Sources: GOC:mah, GOC:rb Relationships: is a type of proteasome-mediated ubiquitin-dependent protein catabolic process [GO:0043161]